{
  "term_label": "extracellular space",
  "gene": "UniProtKB:Q6UY13",
  "gene_symbol": "UNQ5830/PRO19650/PRO19816",
  "gene_name": "Putative uncharacterized protein UNQ5830_PRO19650_PRO19816",
  "term_id": "GO:0005615"
}